chaperone-mediated autophagy translocation complex disassembly [GO:1904764] (biological process) Also known as: CMA translocation complex disassembly, CMA receptor complex disassembly, chaperone-mediated autophagy receptor complex disassembly Definition: The disaggregation of a chaperone-mediated autophagy translocation complex into its constituent components. References: PMID:18644871 Sources: GOC:PARL, GOC:TermGenie, GOC:pad, GO_REF:0000079 Relationships: is a type of protein-containing complex disassembly [GO:0032984]